23S rRNA pseudouridine(955/2504/2580) synthase activity [GO:0160141] (molecular function) Definition: Catalysis of the reaction: uridine(955/2504/2580) in 23S rRNA = pseudouridine(955/2504/2580) in 23S rRNA. Sources: EC:5.4.99.24, RHEA:42528 Relationships: is a type of rRNA pseudouridine synthase activity [GO:0120159]